{
  "gene": "UniProtKB:Q9Y5B0",
  "term_id": "UNKNOWN:0002",
  "gene_symbol": "CTDP1",
  "gene_name": "RNA polymerase II subunit A C-terminal domain phosphatase",
  "term_label": "Unknown biological process"
}